{
  "gene_name": "Acyl-CoA (8-3)-desaturase",
  "term_id": "GO:0016020",
  "gene_symbol": "FADS1",
  "term_label": "membrane",
  "gene": "UniProtKB:O60427"
}